{
  "term_id": "GO:0042573",
  "gene_name": "All-trans-retinol dehydrogenase [NAD(+)] ADH7",
  "term_label": "retinoic acid metabolic process",
  "gene_symbol": "ADH7",
  "gene": "UniProtKB:P40394"
}